{
  "gene": "UniProtKB:Q9BSI4",
  "term_label": "telomere capping",
  "term_id": "GO:0016233",
  "gene_name": "TERF1-interacting nuclear factor 2",
  "gene_symbol": "TINF2"
}